{
  "term_id": "UNKNOWN:0003",
  "gene_symbol": "Q6ZWC4",
  "term_label": "Unknown cellular component",
  "gene": "UniProtKB:Q6ZWC4",
  "gene_name": "Putative uncharacterized protein LOC100128429"
}